{
  "gene": "UniProtKB:A0A0A6YYK7",
  "term_id": "UNKNOWN:0001",
  "gene_symbol": "TRAV19",
  "term_label": "Unknown molecular function",
  "gene_name": "T cell receptor alpha variable 19"
}